{
  "gene": "UniProtKB:Q7Z794",
  "term_id": "GO:0031424",
  "gene_symbol": "KRT77",
  "term_label": "keratinization",
  "gene_name": "Keratin, type II cytoskeletal 1b"
}